{
  "gene": "UniProtKB:Q8NFF2",
  "term_id": "GO:0006874",
  "term_label": "intracellular calcium ion homeostasis",
  "gene_symbol": "SLC24A4",
  "gene_name": "Sodium_potassium_calcium exchanger 4"
}